killing of cells of another organism [GO:0031640] (biological process) Regulation: regulated by regulation of killing of cells of another organism [GO:0051709]; negatively regulated by GO:0051711; positively regulated by positive regulation of killing of cells of another organism [GO:0051712] Relationships: is a type of GO:0001906; is_a disruption of cell in another organism [GO:0141061] Subtypes: GO:0001907, venom-mediated myocyte killing in another organism [GO:0044522], cytolysis in another organism [GO:0051715], killing by host of symbiont cells [GO:0051873] Definition: Any process in an organism that results in the killing of cells of another organism, including in some cases the death of the other organism. Killing here refers to the induction of death in one cell by another cell, not cell-autonomous death due to internal or other environmental conditions. Sources: GOC:add Also known as: killing of cells of other organism